{
  "term_label": "transmembrane signaling receptor activity",
  "term_id": "GO:0004888",
  "gene": "UniProtKB:Q6BAA4",
  "gene_symbol": "FCRLB",
  "gene_name": "Fc receptor-like B"
}